{
  "term_id": "GO:0042393",
  "term_label": "histone binding",
  "gene_name": "WD repeat-containing protein 5B",
  "gene_symbol": "WDR5B",
  "gene": "UniProtKB:Q86VZ2"
}